{
  "term_label": "Unknown biological process",
  "gene_name": "B-cell CLL_lymphoma 7 protein family member B",
  "gene_symbol": "BCL7B",
  "gene": "UniProtKB:Q9BQE9",
  "term_id": "UNKNOWN:0002"
}